S-methylmethionine transmembrane transporter activity [GO:0000100] (molecular function) Also known as: S-methylmethionine transporter activity, S-methylmethionine permease activity Definition: Enables the transfer of S-methylmethionine from one side of a membrane to the other. Relationships: is a type of modified amino acid transmembrane transporter activity [GO:0072349]; is a type of sulfur compound transmembrane transporter activity [GO:1901682]; BFO_0000050 S-methylmethionine transport [GO:0015806] Sources: GOC:ai